{
  "term_label": "Unknown cellular component",
  "gene": "UniProtKB:Q9NZC7",
  "gene_name": "WW domain-containing oxidoreductase",
  "term_id": "UNKNOWN:0003",
  "gene_symbol": "WWOX"
}